{
  "term_id": "UNKNOWN:0002",
  "gene_symbol": "RNLS",
  "term_label": "Unknown biological process",
  "gene_name": "Renalase",
  "gene": "UniProtKB:Q5VYX0"
}